{
  "term_id": "GO:0031463",
  "gene_name": "Ectoderm-neural cortex protein 1",
  "gene_symbol": "ENC1",
  "term_label": "Cul3-RING ubiquitin ligase complex",
  "gene": "UniProtKB:O14682"
}